{
  "term_label": "ATPase-coupled transmembrane transporter activity",
  "term_id": "GO:0042626",
  "gene": "UniProtKB:P78363",
  "gene_name": "Retinal-specific phospholipid-transporting ATPase ABCA4",
  "gene_symbol": "ABCA4"
}